{
  "gene_name": "Tyrosine-protein kinase FRK",
  "gene": "UniProtKB:P42685",
  "gene_symbol": "FRK",
  "term_id": "GO:0030154",
  "term_label": "cell differentiation"
}